positive regulation of meiotic cell cycle process involved in oocyte maturation [GO:1904146] (biological process) Definition: Any process that activates or increases the frequency, rate or extent of meiotic cell cycle process involved in oocyte maturation. Also known as: up regulation of meiotic cell cycle process involved in oocyte maturation, up-regulation of meiotic cell cycle process involved in oocyte maturation, upregulation of meiotic cell cycle process involved in oocyte maturation, activation of meiotic cell cycle process involved in oocyte maturation Relationships: is a type of GO:0051446; is_a positive regulation of cell cycle process [GO:0090068]; is a type of regulation of meiotic cell cycle process involved in oocyte maturation [GO:1903538]; positively regulates GO:1903537 References: PMID:22674394 Sources: GOC:TermGenie, GO_REF:0000058